{
  "gene_name": "NF-kappa-B-repressing factor",
  "gene": "UniProtKB:O15226",
  "gene_symbol": "NKRF",
  "term_label": "RNA polymerase II cis-regulatory region sequence-specific DNA binding",
  "term_id": "GO:0000978"
}